glycine betaine biosynthetic process from choline [GO:0019285] (biological process) Also known as: N-trimethylglycine biosynthesis from choline, N-trimethylglycine biosynthetic process from choline, choline oxidation, glycine betaine anabolism from choline, glycine betaine formation from choline, glycine betaine synthesis from choline Definition: The chemical reactions and pathways resulting in the formation of betaine (N-trimethylglycine) from the oxidation of choline. Sources: GOC:jl Relationships: is a type of GO:0019695; is a type of GO:0031456